{
  "gene": "UniProtKB:O14787",
  "term_label": "protein import into nucleus",
  "gene_name": "Transportin-2",
  "gene_symbol": "TNPO2",
  "term_id": "GO:0006606"
}